{
  "gene_name": "Cysteine-rich protein 1",
  "gene": "UniProtKB:P50238",
  "gene_symbol": "CRIP1",
  "term_label": "regulation of gene expression",
  "term_id": "GO:0010468"
}